NADPH-iron-sulfur [2Fe-2S] protein oxidoreductase activity [GO:0160246] (molecular function) Definition: Catalysis of the reaction: 2 oxidized [2Fe-2S]-[protein] + NADPH = 2 reduced [2Fe-2S]-[protein] + NADP+ + H+. Sources: RHEA:67716 Relationships: is a type of oxidoreductase activity, acting on iron-sulfur proteins as donors, NAD or NADP as acceptor [GO:0016731]